pseudocleavage involved in syncytial blastoderm formation [GO:0030589] (BP) Relationships: is a type of GO:0030588; is part of embryonic development via the syncytial blastoderm [GO:0001700] Also known as: pseudocleavage during syncytial blastoderm formation Sources: GOC:mtg_sensu Definition: Formation of furrows in the cytoplasm between nuclei during cell cycles in embryos that contribute to the formation of the syncytial blastoderm. An example of this process is found in Drosophila melanogaster.